{
  "term_id": "GO:0007265",
  "term_label": "Ras protein signal transduction",
  "gene_symbol": "RASGEF1B",
  "gene_name": "Ras-GEF domain-containing family member 1B",
  "gene": "UniProtKB:Q0VAM2"
}